{
  "gene_symbol": "HRG",
  "term_id": "GO:0005576",
  "term_label": "extracellular region",
  "gene": "UniProtKB:P04196",
  "gene_name": "Histidine-rich glycoprotein"
}